RPB4-RPB7 complex [GO:1990328] (cellular component) Relationships: is a type of intracellular protein-containing complex [GO:0140535] References: PMID:15591044 Sources: GOC:bhm Also known as: RNA polymerase II, RPB4-RPB7 subcomplex Definition: A protein complex that cycles between the nucleus where it is part of the RNA polymerase II and the cytoplasmic mRNA processing body where it mediates the two major cytoplasmic mRNA decay pathways.